{
  "term_label": "D-mannose binding",
  "gene_symbol": "CLEC10A",
  "gene_name": "C-type lectin domain family 10 member A",
  "gene": "UniProtKB:Q8IUN9",
  "term_id": "GO:0005537"
}